nuclear polyadenylation-dependent antisense transcript catabolic process [GO:0071040] (biological process) Also known as: nuclear poly(A)-dependent antisense transcript catabolic process Relationships: is a type of GO:0071041 References: PMID:18022365 Sources: GOC:dgf, GOC:krc Definition: The chemical reactions and pathways occurring in the nucleus and resulting in the breakdown of an antisense transcript, initiated by the enzymatic addition of a sequence of adenylyl residues (polyadenylation) at the 3' end the target antisense transcript.